negative regulation of peptidyl-serine phosphorylation [GO:0033137] (biological process) Subtypes: GO:0033140 Definition: Any process that stops, prevents, or reduces the frequency, rate or extent of the phosphorylation of peptidyl-serine. Sources: GOC:mah Relationships: is a type of negative regulation of protein phosphorylation [GO:0001933]; is a type of regulation of peptidyl-serine phosphorylation [GO:0033135]; negatively regulates peptidyl-serine phosphorylation [GO:0018105]